{
  "gene_name": "DnaJ homolog subfamily B member 5",
  "gene": "UniProtKB:O75953",
  "term_id": "GO:0051082",
  "term_label": "unfolded protein binding",
  "gene_symbol": "DNAJB5"
}